{
  "gene": "UniProtKB:P10809",
  "term_id": "GO:0045041",
  "gene_name": "60 kDa heat shock protein, mitochondrial",
  "gene_symbol": "HSPD1",
  "term_label": "protein import into mitochondrial intermembrane space"
}